{
  "term_label": "extracellular matrix structural constituent conferring tensile strength",
  "gene_name": "Collagen alpha-1(XVIII) chain",
  "gene_symbol": "COL18A1",
  "term_id": "GO:0030020",
  "gene": "UniProtKB:P39060"
}